{
  "gene_name": "Olfactory receptor",
  "term_id": "GO:0007186",
  "gene": "UniProtKB:A0A2R8Y4L6",
  "gene_symbol": "OR5D3",
  "term_label": "G protein-coupled receptor signaling pathway"
}